{
  "gene_name": "Chromobox protein homolog 6",
  "gene": "UniProtKB:O95503",
  "term_label": "chromatin",
  "gene_symbol": "CBX6",
  "term_id": "GO:0000785"
}